{
  "gene_symbol": "POLN",
  "gene_name": "DNA polymerase nu",
  "gene": "UniProtKB:Q7Z5Q5",
  "term_id": "GO:0003887",
  "term_label": "DNA-directed DNA polymerase activity"
}